{
  "term_label": "alkenylglycerophosphocholine hydrolase activity",
  "term_id": "GO:0047408",
  "gene": "UniProtKB:Q8N661",
  "gene_name": "Lysoplasmalogenase",
  "gene_symbol": "TMEM86B"
}